{
  "term_id": "GO:0005634",
  "gene_name": "Nuclear factor 1 X-type",
  "gene": "UniProtKB:Q14938",
  "gene_symbol": "NFIX",
  "term_label": "nucleus"
}